{
  "term_label": "signaling receptor activity",
  "gene_symbol": "NLGN3",
  "gene_name": "Neuroligin-3",
  "gene": "UniProtKB:Q9NZ94",
  "term_id": "GO:0038023"
}